{
  "term_id": "GO:0000978",
  "gene": "UniProtKB:Q6ECI4",
  "gene_name": "Zinc finger protein 470",
  "gene_symbol": "ZNF470",
  "term_label": "RNA polymerase II cis-regulatory region sequence-specific DNA binding"
}